{
  "term_label": "Unknown molecular function",
  "gene": "UniProtKB:Q5GH73",
  "gene_name": "XK-related protein 6",
  "term_id": "UNKNOWN:0001",
  "gene_symbol": "XKR6"
}